dihydrostreptomycin-6-phosphate 3'-alpha-kinase activity [GO:0047333] (molecular function) Definition: Catalysis of the reaction: ATP + dihydrostreptomycin 6-phosphate = ADP + dihydrostreptomycin 3'alpha,6-bisphosphate + 2 H+. Relationships: is a type of aminoglycoside phosphotransferase activity [GO:0034071] Also known as: ATP:dihydrostreptomycin-6-P 3'alpha-phosphotransferase activity, ATP:dihydrostreptomycin-6-phosphate 3'alpha-phosphotransferase activity, dihydrostreptomycin 6-phosphate kinase (phosphorylating), dihydrostreptomycin-6-phosphate 3'alpha-kinase activity Sources: EC:2.7.1.88, RHEA:16281